{
  "term_id": "GO:0016887",
  "term_label": "ATP hydrolysis activity",
  "gene": "UniProtKB:P46459",
  "gene_symbol": "NSF",
  "gene_name": "Vesicle-fusing ATPase"
}